{
  "gene": "UniProtKB:Q9UHD2",
  "term_id": "GO:0005737",
  "term_label": "cytoplasm",
  "gene_name": "Serine_threonine-protein kinase TBK1",
  "gene_symbol": "TBK1"
}